{
  "gene_name": "DNA-directed primase_polymerase protein",
  "gene_symbol": "PRIMPOL",
  "term_label": "response to UV",
  "gene": "UniProtKB:Q96LW4",
  "term_id": "GO:0009411"
}